{
  "term_label": "microtubule associated complex",
  "gene": "UniProtKB:Q14203",
  "term_id": "GO:0005875",
  "gene_name": "Dynactin subunit 1",
  "gene_symbol": "DCTN1"
}